{
  "term_label": "Unknown cellular component",
  "gene_name": "Chromosome 6 open reading frame 48, isoform CRA_a",
  "gene": "UniProtKB:A0A024RCN7",
  "gene_symbol": "SNHG32",
  "term_id": "UNKNOWN:0003"
}